{
  "gene_name": "Threonine--tRNA ligase 1, cytoplasmic",
  "gene_symbol": "TARS1",
  "term_label": "cytoplasm",
  "gene": "UniProtKB:P26639",
  "term_id": "GO:0005737"
}